bacterial-type flagellum basal body, distal rod, P ring [GO:0009428] (cellular component) References: PMID:10572114, PMID:12624192 Sources: GOC:cilia, GOC:mtg_sensu Definition: One of the rings of the bacterial-type flagellar basal body; anchors the basal body to the peptidoglycan layer. Relationships: is a type of cellular anatomical structure [GO:0110165]; is part of bacterial-type flagellum basal body, distal rod [GO:0009426] Also known as: flagellin-based flagellum basal body, distal rod, P ring, flagellar basal body, distal rod, P ring